{
  "gene_name": "FERM and PDZ domain-containing protein 4",
  "gene": "UniProtKB:Q14CM0",
  "term_id": "UNKNOWN:0002",
  "gene_symbol": "FRMPD4",
  "term_label": "Unknown biological process"
}